{
  "gene_symbol": "DCUN1D1",
  "term_id": "GO:0045116",
  "gene_name": "DCN1-like protein 1",
  "term_label": "protein neddylation",
  "gene": "UniProtKB:Q96GG9"
}